{
  "term_label": "catenin complex",
  "term_id": "GO:0016342",
  "gene_symbol": "APC",
  "gene": "UniProtKB:P25054",
  "gene_name": "Adenomatous polyposis coli protein"
}